DNA ADP-ribosylation [GO:0030592] (biological process) Relationships: is_a DNA modification [GO:0006304] Definition: The covalent attachment of an ADP-ribosyl group to a residue in double-stranded DNA. References: PMID:11592983, PMID:27471034, PMID:29361132, PMID:29520010